{
  "gene_name": "Kinesin-like protein KIF25",
  "term_label": "kinesin complex",
  "gene": "UniProtKB:Q9UIL4",
  "term_id": "GO:0005871",
  "gene_symbol": "KIF25"
}